positive regulation of anthocyanin catabolic process [GO:1900002] (biological process) Definition: Any process that activates or increases the frequency, rate or extent of anthocyanin catabolic process. Relationships: is a type of positive regulation of catabolic process [GO:0009896]; is a type of positive regulation of anthocyanin metabolic process [GO:0031539]; is a type of GO:1900000; positively regulates anthocyanin-containing compound catabolic process [GO:0046284] Also known as: positive regulation of anthocyanin breakdown, positive regulation of anthocyanin catabolism, positive regulation of anthocyanin degradation, up regulation of anthocyanin breakdown, up regulation of anthocyanin catabolism, up regulation of anthocyanin degradation, up regulation of anthocyanin catabolic process Sources: GOC:TermGenie